{
  "gene_symbol": "LOC122539214",
  "term_id": "GO:0006357",
  "gene": "UniProtKB:A0A7P0TAN4",
  "term_label": "regulation of transcription by RNA polymerase II",
  "gene_name": "Uncharacterized protein"
}